L-seryl-tRNA(Thr) hydrolase activity [GO:0043905] (molecular function) Also known as: Ser-tRNA(Thr) hydrolase activity, Ser-tRNAThr hydrolase activity Definition: Catalysis of the hydrolysis of misacylated Ser-tRNA(Thr). Relationships: is_a carboxylic ester hydrolase activity [GO:0052689]; is a type of catalytic activity, acting on a tRNA [GO:0140101] References: PMID:15240874 Sources: GOC:jl